uridine kinase activity [GO:0004849] (molecular function) Definition: Catalysis of the reaction: ATP + uridine = ADP + UMP. Sources: RHEA:16825 Also known as: uridine phosphokinase activity, uridine-cytidine kinase activity Relationships: is a type of GO:0019206; is part of UMP biosynthetic process [GO:0006222]